blood coagulation [GO:0007596] (biological process) Regulation: RO_0002211 by regulation of blood coagulation [GO:0030193]; RO_0002213 by positive regulation of blood coagulation [GO:0030194]; negatively regulated by GO:0030195 Also known as: blood clotting Definition: The sequential process in which the multiple coagulation factors of the blood interact, ultimately resulting in the formation of an insoluble fibrin clot; it may be divided into three stages: stage 1, the formation of intrinsic and extrinsic prothrombin converting principle; stage 2, the formation of thrombin; stage 3, the formation of stable fibrin polymers. References: PMID:30700128 Relationships: is a type of hemostasis [GO:0007599]; is a type of coagulation [GO:0050817]; is part of wound healing [GO:0042060]